{
  "gene_name": "Cadherin-1",
  "gene_symbol": "CDH1",
  "gene": "UniProtKB:P12830",
  "term_id": "GO:0045296",
  "term_label": "cadherin binding"
}